{
  "gene_name": "E3 ubiquitin-protein ligase TRIM9",
  "term_id": "UNKNOWN:0002",
  "gene_symbol": "TRIM9",
  "term_label": "Unknown biological process",
  "gene": "UniProtKB:Q9C026"
}